{
  "term_id": "GO:0061630",
  "gene": "UniProtKB:A6NLI5",
  "gene_symbol": "TRIM64C",
  "gene_name": "Tripartite motif-containing protein 64C",
  "term_label": "ubiquitin protein ligase activity"
}